{
  "term_label": "Unknown molecular function",
  "gene_name": "Cordon-bleu protein-like 1",
  "gene": "UniProtKB:Q53SF7",
  "term_id": "UNKNOWN:0001",
  "gene_symbol": "COBLL1"
}